{
  "term_id": "GO:0050852",
  "term_label": "T cell receptor signaling pathway",
  "gene_symbol": "LAT",
  "gene_name": "Linker for activation of T-cells family member 1",
  "gene": "UniProtKB:O43561"
}